{
  "gene": "UniProtKB:Q92922",
  "term_label": "nBAF complex",
  "gene_symbol": "SMARCC1",
  "term_id": "GO:0071565",
  "gene_name": "SWI_SNF complex subunit SMARCC1"
}